positive regulation of protein localization to meiotic spindle pole body [GO:0140434] (biological process) Definition: Any process that increases the frequency, rate or extent of protein localization to a meiotic spindle pole body. Relationships: is a type of GO:0140433; is a type of positive regulation of protein localization to spindle pole body [GO:1902365]; positively regulates protein localization to meiotic spindle pole body [GO:1902441] References: PMID:22438582